extrinsic component of external side of mycolate outer membrane [GO:0036421] (cellular component) Also known as: extrinsic to external side of MOM, extrinsic to external side of mycomembrane, extrinsic to external side of mycolate outer membrane Sources: GOC:md Relationships: is a type of extrinsic component of external side of cell outer membrane [GO:0031242]; is_a extrinsic component of mycolate outer membrane [GO:0036420]; is part of external side of mycolate outer membrane [GO:0098568] Definition: The component of mycolate membrane consisting of gene products and protein complexes that are loosely bound to its external surface, but not integrated into the hydrophobic region.